{
  "gene_symbol": "PPP2R3B",
  "gene_name": "Serine_threonine-protein phosphatase 2A regulatory subunit B'' subunit beta",
  "gene": "UniProtKB:Q9Y5P8",
  "term_id": "GO:0000159",
  "term_label": "protein phosphatase type 2A complex"
}